{
  "gene_name": "Guanine nucleotide exchange factor VAV3",
  "gene": "UniProtKB:Q9UKW4",
  "term_label": "immune response-regulating cell surface receptor signaling pathway",
  "gene_symbol": "VAV3",
  "term_id": "GO:0002768"
}